xylem development [GO:0010089] (biological process) Definition: The formation of the principal water-conducting tissue of a vascular plant. Relationships: is a type of phloem or xylem histogenesis [GO:0010087] Also known as: xylem histogenesis Sources: GOC:tb, ISBN:0471245208 Subtypes: metaxylem development [GO:0090058], protoxylem development [GO:0090059]